{
  "gene_name": "1-phosphatidylinositol 4,5-bisphosphate phosphodiesterase beta-1",
  "gene": "UniProtKB:Q9NQ66",
  "term_id": "GO:0007186",
  "gene_symbol": "PLCB1",
  "term_label": "G protein-coupled receptor signaling pathway"
}